{
  "gene": "UniProtKB:Q92832",
  "term_label": "regulation of osteoblast differentiation",
  "gene_name": "Protein kinase C-binding protein NELL1",
  "term_id": "GO:0045667",
  "gene_symbol": "NELL1"
}